{
  "term_id": "GO:0033539",
  "gene": "UniProtKB:Q6JQN1",
  "term_label": "fatty acid beta-oxidation using acyl-CoA dehydrogenase",
  "gene_name": "Acyl-CoA dehydrogenase family member 10",
  "gene_symbol": "ACAD10"
}